{
  "term_label": "RNA polymerase II complex binding",
  "gene": "UniProtKB:O94913",
  "gene_symbol": "PCF11",
  "gene_name": "Pre-mRNA cleavage complex 2 protein Pcf11",
  "term_id": "GO:0000993"
}